{
  "gene": "UniProtKB:Q96SI9",
  "term_id": "GO:0003725",
  "gene_symbol": "STRBP",
  "gene_name": "Spermatid perinuclear RNA-binding protein",
  "term_label": "double-stranded RNA binding"
}